{
  "term_label": "endoplasmic reticulum exit site",
  "term_id": "GO:0070971",
  "gene": "UniProtKB:Q15436",
  "gene_symbol": "SEC23A",
  "gene_name": "Protein transport protein Sec23A"
}